{
  "term_label": "G protein-coupled receptor activity",
  "gene_symbol": "FFAR4",
  "term_id": "GO:0004930",
  "gene_name": "Free fatty acid receptor 4",
  "gene": "UniProtKB:Q5NUL3"
}